{
  "gene": "UniProtKB:O14561",
  "gene_name": "Acyl carrier protein, mitochondrial",
  "gene_symbol": "NDUFAB1",
  "term_label": "acyl carrier activity",
  "term_id": "GO:0000036"
}